{
  "gene_name": "T cell receptor beta variable 12-4",
  "term_id": "UNKNOWN:0001",
  "gene": "UniProtKB:A0A0B4J2E0",
  "term_label": "Unknown molecular function",
  "gene_symbol": "TRBV12-4"
}